{
  "gene": "UniProtKB:P82933",
  "term_id": "GO:0005763",
  "gene_symbol": "MRPS9",
  "gene_name": "Small ribosomal subunit protein uS9m",
  "term_label": "mitochondrial small ribosomal subunit"
}